{
  "term_id": "GO:0000723",
  "term_label": "telomere maintenance",
  "gene_name": "DNA repair protein RAD51 homolog 4",
  "gene_symbol": "RAD51D",
  "gene": "UniProtKB:O75771"
}